{
  "gene_name": "Anoctamin-5",
  "term_id": "GO:0045332",
  "term_label": "phospholipid translocation",
  "gene": "UniProtKB:Q75V66",
  "gene_symbol": "ANO5"
}